{
  "gene_symbol": "TCIRG1",
  "term_id": "GO:0007035",
  "gene": "UniProtKB:Q13488",
  "gene_name": "V-type proton ATPase 116 kDa subunit a 3",
  "term_label": "vacuolar acidification"
}